{
  "gene_name": "Thrombospondin-1",
  "term_id": "UNKNOWN:0001",
  "gene_symbol": "THBS1",
  "gene": "UniProtKB:P07996",
  "term_label": "Unknown molecular function"
}